{
  "term_label": "phospholipid binding",
  "gene_name": "Putative synaptotagmin-14-like protein",
  "gene": "UniProtKB:Q58G82",
  "gene_symbol": "SYT14P1",
  "term_id": "GO:0005543"
}